{
  "gene_symbol": "HSP90AB2P",
  "gene": "UniProtKB:Q58FF8",
  "term_id": "GO:0032991",
  "gene_name": "Putative heat shock protein HSP 90-beta 2",
  "term_label": "protein-containing complex"
}